{
  "term_id": "GO:0004714",
  "gene": "UniProtKB:P21709",
  "term_label": "transmembrane receptor protein tyrosine kinase activity",
  "gene_symbol": "EPHA1",
  "gene_name": "Ephrin type-A receptor 1"
}